{
  "gene_symbol": "PLGLA",
  "term_label": "Unknown biological process",
  "term_id": "UNKNOWN:0002",
  "gene_name": "Plasminogen-like protein A",
  "gene": "UniProtKB:Q15195"
}